{
  "gene": "UniProtKB:A2RUC4",
  "gene_symbol": "TYW5",
  "term_label": "tRNA(Phe) (7-(3-amino-3-carboxypropyl)wyosine37-C2)-hydroxylase activity",
  "term_id": "GO:0102524",
  "gene_name": "tRNA wybutosine-synthesizing protein 5"
}